{
  "gene_symbol": "SRFBP1",
  "gene_name": "Serum response factor-binding protein 1",
  "term_id": "GO:0005634",
  "gene": "UniProtKB:Q8NEF9",
  "term_label": "nucleus"
}